{
  "gene_name": "Zinc finger protein 761",
  "term_label": "RNA polymerase II cis-regulatory region sequence-specific DNA binding",
  "gene": "UniProtKB:Q86XN6",
  "gene_symbol": "ZNF761",
  "term_id": "GO:0000978"
}